{
  "term_id": "GO:0009922",
  "gene_name": "Elongation of very long chain fatty acids protein 1",
  "gene": "UniProtKB:Q9BW60",
  "term_label": "fatty acid elongase activity",
  "gene_symbol": "ELOVL1"
}